{
  "gene_name": "Glutamate receptor 1",
  "gene": "UniProtKB:P42261",
  "term_id": "GO:0005886",
  "term_label": "plasma membrane",
  "gene_symbol": "GRIA1"
}